{
  "term_label": "Unknown molecular function",
  "term_id": "UNKNOWN:0001",
  "gene": "UniProtKB:Q0D2H9",
  "gene_name": "Putative golgin subfamily A member 8D",
  "gene_symbol": "GOLGA8DP"
}